{
  "gene": "UniProtKB:Q9NUQ6",
  "term_label": "Unknown biological process",
  "gene_name": "SPATS2-like protein",
  "gene_symbol": "SPATS2L",
  "term_id": "UNKNOWN:0002"
}